{
  "gene": "UniProtKB:C9JQL5",
  "gene_symbol": "C9JQL5",
  "term_id": "GO:0005886",
  "term_label": "plasma membrane",
  "gene_name": "Putative dispanin subfamily A member 2d"
}